{
  "term_label": "cell adhesion",
  "term_id": "GO:0007155",
  "gene": "UniProtKB:Q14773",
  "gene_name": "Intercellular adhesion molecule 4",
  "gene_symbol": "ICAM4"
}